{
  "gene_name": "T cell receptor beta variable 10-1",
  "gene_symbol": "TRBV10-1",
  "gene": "UniProtKB:A0A0K0K1A3",
  "term_label": "plasma membrane",
  "term_id": "GO:0005886"
}